{
  "term_label": "Unknown molecular function",
  "gene_symbol": "GIG44",
  "gene": "UniProtKB:P09565",
  "term_id": "UNKNOWN:0001",
  "gene_name": "Putative insulin-like growth factor 2-associated protein"
}